{
  "term_label": "nucleus",
  "gene_name": "Interferon-stimulated 20 kDa exonuclease-like 2",
  "term_id": "GO:0005634",
  "gene_symbol": "ISG20L2",
  "gene": "UniProtKB:Q9H9L3"
}